{
  "gene": "UniProtKB:Q16773",
  "gene_symbol": "KYAT1",
  "term_label": "Unknown biological process",
  "term_id": "UNKNOWN:0002",
  "gene_name": "Kynurenine--oxoglutarate transaminase 1"
}